protein C inhibitor-coagulation factor Xa complex [GO:0097182] (cellular component) Also known as: PCI-coagulation factor Xa complex, SERPINA5-coagulation factor Xa complex, plasma serine protease inhibitor-coagulation factor Xa complex, serpin A5-coagulation factor Xa complex References: PMID:6323392 Sources: GOC:ans Definition: A heterodimeric protein complex that contains protein C inhibitor (SERPINA5) and coagulation factor Xa (F10); formation of the complex inhibits the serine protease activity of coagulation factor Xa. Relationships: is a type of serine protease inhibitor complex [GO:0097180]